{
  "gene_symbol": "RABGAP1L",
  "term_label": "regulation of protein localization",
  "gene_name": "Rab GTPase-activating protein 1-like",
  "term_id": "GO:0032880",
  "gene": "UniProtKB:Q5R372"
}